{
  "term_label": "positive regulation of DNA-templated transcription, elongation",
  "gene_symbol": "CCNT2",
  "gene": "UniProtKB:O60583",
  "gene_name": "Cyclin-T2",
  "term_id": "GO:0032786"
}